{
  "gene_name": "Olfactory receptor 5C1",
  "term_id": "UNKNOWN:0002",
  "term_label": "Unknown biological process",
  "gene_symbol": "OR5C1",
  "gene": "UniProtKB:Q8NGR4"
}